{
  "term_label": "determination of left/right symmetry",
  "gene": "UniProtKB:P0CG36",
  "gene_symbol": "CFC1B",
  "term_id": "GO:0007368",
  "gene_name": "Cryptic family protein 1B"
}